{
  "term_id": "UNKNOWN:0002",
  "gene_name": "Protein FAM228B",
  "gene": "UniProtKB:P0C875",
  "gene_symbol": "FAM228B",
  "term_label": "Unknown biological process"
}